{
  "term_label": "negative regulation of growth hormone receptor signaling pathway",
  "gene_name": "Leptin receptor gene-related protein",
  "gene": "UniProtKB:O15243",
  "term_id": "GO:0060400",
  "gene_symbol": "LEPROT"
}